{
  "term_id": "UNKNOWN:0001",
  "term_label": "Unknown molecular function",
  "gene_symbol": "MFSD4B",
  "gene_name": "Sodium-dependent glucose transporter 1",
  "gene": "UniProtKB:Q5TF39"
}